entry into dormancy [GO:0097436] (biological process) Also known as: induction of dormancy Sources: GOC:PO_curators, PO_REF:00009 Relationships: is a type of dormancy process [GO:0022611] Definition: The dormancy process that results in entry into dormancy. Dormancy (sometimes called a dormant state) is a suspension of most physiological activity and growth that can be reactivated.